prostanoid receptor binding [GO:0031862] (molecular function) Relationships: is_a G protein-coupled receptor binding [GO:0001664] Also known as: prostanoid receptor ligand Definition: Binding to a prostanoid receptor. Sources: GOC:mah, GOC:nln Subtypes: GO:0031863, GO:0031864, GO:0031865, GO:0031866, GO:0031867, prostaglandin F2-alpha receptor binding [GO:0031868], prostacyclin receptor binding [GO:0031869], GO:0031870